{
  "gene": "UniProtKB:A6NI15",
  "gene_name": "Mesogenin-1",
  "gene_symbol": "MSGN1",
  "term_label": "regulation of transcription by RNA polymerase II",
  "term_id": "GO:0006357"
}